pyridine nucleotide catabolic process [GO:0019364] (biological process) Relationships: is a type of GO:0009166; is_a pyridine-containing compound catabolic process [GO:0072526] Subtypes: glycolytic process [GO:0006096], NADP+ catabolic process [GO:0006742], NAD+ catabolic process [GO:0019677] Definition: The chemical reactions and pathways resulting in the breakdown of a pyridine nucleotide, a nucleotide characterized by a pyridine derivative as a nitrogen base. Also known as: pyridine nucleotide breakdown, pyridine nucleotide catabolism, pyridine nucleotide degradation Sources: GOC:jl, GOC:pde, GOC:vw